{
  "gene": "UniProtKB:P50549",
  "gene_name": "ETS translocation variant 1",
  "term_label": "regulation of transcription by RNA polymerase II",
  "term_id": "GO:0006357",
  "gene_symbol": "ETV1"
}